response to isoquinoline alkaloid [GO:0014072] (biological process) Definition: Any process that results in a change in state or activity of a cell or an organism (in terms of movement, secretion, enzyme production, gene expression, etc.) as a result of an isoquinoline alkaloid stimulus. An isoquinoline alkaloid is any member of a group of compounds with the heterocyclic ring structure of benzo(c)pyridine which is a structure characteristic of the group of opium alkaloids. Subtypes: GO:0043278, cellular response to isoquinoline alkaloid [GO:0071317], response to dextromethorphan [GO:1904558], GO:1905233 Sources: GOC:ef Relationships: is a type of response to alkaloid [GO:0043279]